{
  "term_label": "transcription corepressor activity",
  "gene_name": "Testis-specific chromodomain protein Y 2",
  "gene_symbol": "CDY2A",
  "term_id": "GO:0003714",
  "gene": "UniProtKB:Q9Y6F7"
}